positive regulation of establishment of protein localization to telomere [GO:1904851] (biological process) Also known as: positive regulation of establishment of protein localisation to telomere, positive regulation of establishment of protein localization to chromosome, telomeric region, up regulation of establishment of protein localisation to telomere, up regulation of establishment of protein localization to chromosome, telomeric region, up regulation of establishment of protein localization to telomere, up-regulation of establishment of protein localisation to telomere, up-regulation of establishment of protein localization to chromosome, telomeric region, up-regulation of establishment of protein localization to telomere, upregulation of establishment of protein localisation to telomere, upregulation of establishment of protein localization to chromosome, telomeric region, upregulation of establishment of protein localization to telomere, activation of establishment of protein localisation to telomere, activation of establishment of protein localization to chromosome, telomeric region, activation of establishment of protein localization to telomere References: PMID:25467444 Sources: GOC:BHF, GOC:BHF_telomere, GOC:TermGenie, GOC:nc, GO_REF:0000058 Definition: Any process that activates or increases the frequency, rate or extent of establishment of protein localization to telomere. Relationships: is a type of regulation of establishment of protein localization to telomere [GO:0070203]; is a type of GO:1904951; positively regulates GO:0070200